non-glycolytic fermentation [GO:0019662] (biological process) Sources: GOC:jl Definition: Fermentation that does not include the anaerobic conversion of glucose to pyruvate via the glycolytic pathway. Subtypes: GO:0019588, citrate catabolic process to diacetyl [GO:0019651], lactate fermentation to propionate and acetate [GO:0019652], glucose catabolic process to D-lactate and ethanol [GO:0019656], glucose fermentation to lactate and acetate [GO:0019658], GO:0019672 Relationships: is a type of GO:0006113